{
  "gene_name": "Leucine-zipper-like transcriptional regulator 1",
  "term_id": "UNKNOWN:0001",
  "gene": "UniProtKB:Q8N653",
  "gene_symbol": "LZTR1",
  "term_label": "Unknown molecular function"
}